{
  "gene": "UniProtKB:Q9HCE0",
  "gene_name": "Ectopic P granules protein 5 homolog",
  "term_id": "GO:0005737",
  "term_label": "cytoplasm",
  "gene_symbol": "EPG5"
}